{
  "term_label": "nucleus",
  "gene_symbol": "PADI6",
  "gene_name": "Protein-arginine deiminase type-6",
  "term_id": "GO:0005634",
  "gene": "UniProtKB:Q6TGC4"
}